{
  "gene_symbol": "UFL1",
  "term_label": "response to endoplasmic reticulum stress",
  "gene_name": "E3 UFM1-protein ligase 1",
  "term_id": "GO:0034976",
  "gene": "UniProtKB:O94874"
}